{
  "gene_symbol": "NXPH1",
  "gene": "UniProtKB:P58417",
  "gene_name": "Neurexophilin-1",
  "term_id": "GO:0005102",
  "term_label": "signaling receptor binding"
}